{
  "gene_symbol": "ANAPC15",
  "gene_name": "Anaphase-promoting complex subunit 15",
  "term_label": "anaphase-promoting complex",
  "term_id": "GO:0005680",
  "gene": "UniProtKB:P60006"
}